{
  "gene_symbol": "SELE",
  "gene_name": "E-selectin",
  "gene": "UniProtKB:P16581",
  "term_label": "external side of plasma membrane",
  "term_id": "GO:0009897"
}